chromatin lock complex [GO:0061793] (cellular component) Relationships: is a type of chromatin silencing complex [GO:0005677] References: PMID:17540172 Sources: GOC:bhm, GOC:dph Definition: A chromatin silencing complex that binds and bridges separate nucleosomal histones resulting in heterochromatin assembly and chromatin looping. Also known as: nucleosome bridging complex